regulation of cell morphogenesis involved in phenotypic switching [GO:1900447] (biological process) Sources: GOC:TermGenie, GOC:di Relationships: is a type of regulation of cell morphogenesis [GO:0022604]; is part of phenotypic switching [GO:0036166] Definition: Any process that modulates the frequency, rate or extent of cell morphogenesis contributing a phenotypic switch. Cell morphogenesis involved in differentiation is the change in form (cell shape and size) that occurs when relatively unspecialized cells, such as the opaque cells of C. albicans, acquire specialized structural and/or functional features that characterize the cells, tissues, or organs of the mature organism or some other relatively stable phase of the organism's life history. Also known as: regulation of cell morphogenesis of phenotypic switching, negative regulation of cell shape and cell size of phenotypic dimorphism, negative regulation of cell shape and cell size of phenotypic switching, positive regulation of cell shape and cell size of phenotypic dimorphism, positive regulation of cell shape and cell size of phenotypic switching, regulation of cell morphogenesis of phenotypic dimorphism, regulation of cell shape and cell size of phenotypic dimorphism, regulation of cell shape and cell size of phenotypic switching